{
  "term_id": "GO:0071786",
  "gene": "UniProtKB:Q9C0E8",
  "gene_symbol": "LNPK",
  "term_label": "endoplasmic reticulum tubular network organization",
  "gene_name": "Endoplasmic reticulum junction formation protein lunapark"
}